{
  "term_id": "GO:0000932",
  "term_label": "P-body",
  "gene": "UniProtKB:Q58A45",
  "gene_name": "PAN2-PAN3 deadenylation complex subunit PAN3",
  "gene_symbol": "PAN3"
}